{
  "gene_name": "Fibrillin-1",
  "term_id": "GO:0006006",
  "term_label": "glucose metabolic process",
  "gene": "UniProtKB:P35555",
  "gene_symbol": "FBN1"
}